{
  "term_id": "GO:0045202",
  "gene_name": "Synaptotagmin-11",
  "gene_symbol": "SYT11",
  "term_label": "synapse",
  "gene": "UniProtKB:Q9BT88"
}